{
  "gene_name": "M-phase inducer phosphatase 2",
  "term_id": "GO:0005634",
  "gene": "UniProtKB:P30305",
  "term_label": "nucleus",
  "gene_symbol": "CDC25B"
}